{
  "term_label": "axoneme assembly",
  "term_id": "GO:0035082",
  "gene_symbol": "DNAAF1",
  "gene": "UniProtKB:Q8NEP3",
  "gene_name": "Dynein axonemal assembly factor 1"
}